nuclear pore complex assembly [GO:0051292] (BP) Also known as: NPC assembly, nuclear pore assembly, nuclear pore biogenesis, nuclear pore biosynthesis, nuclear pore complex biogenesis, nuclear pore complex biosynthesis, nuclear pore complex formation, nuclear pore formation Subtypes: mitotic nuclear pore complex reassembly [GO:0007087] Sources: GOC:ai, GOC:mah Relationships: is a type of nuclear pore organization [GO:0006999]; is a type of pore complex assembly [GO:0046931] Definition: The aggregation, arrangement and bonding together of a set of components to form a nuclear pore complex.